negative regulation of tetrapyrrole biosynthetic process from glycine and succinyl-CoA [GO:1901414] (biological process) Sources: GOC:TermGenie, GOC:mengo_curators Also known as: down regulation of tetrapyrrole anabolism from glycine and succinyl-CoA, down regulation of tetrapyrrole biosynthesis from glycine and succinyl-CoA, down regulation of tetrapyrrole biosynthetic process from glycine and succinyl-CoA, down regulation of tetrapyrrole formation from glycine and succinyl-CoA, down regulation of tetrapyrrole synthesis from glycine and succinyl-CoA, down-regulation of tetrapyrrole anabolism from glycine and succinyl-CoA, down-regulation of tetrapyrrole biosynthesis from glycine and succinyl-CoA, down-regulation of tetrapyrrole biosynthetic process from glycine and succinyl-CoA, down-regulation of tetrapyrrole formation from glycine and succinyl-CoA, down-regulation of tetrapyrrole synthesis from glycine and succinyl-CoA, downregulation of tetrapyrrole anabolism from glycine and succinyl-CoA, downregulation of tetrapyrrole biosynthesis from glycine and succinyl-CoA, downregulation of tetrapyrrole biosynthetic process from glycine and succinyl-CoA, downregulation of tetrapyrrole formation from glycine and succinyl-CoA, downregulation of tetrapyrrole synthesis from glycine and succinyl-CoA, inhibition of tetrapyrrole anabolism from glycine and succinyl-CoA, inhibition of tetrapyrrole biosynthesis from glycine and succinyl-CoA, inhibition of tetrapyrrole formation from glycine and succinyl-CoA, inhibition of tetrapyrrole synthesis from glycine and succinyl-CoA, negative regulation of tetrapyrrole anabolism from glycine and succinyl-CoA, negative regulation of tetrapyrrole biosynthesis from glycine and succinyl-CoA, negative regulation of tetrapyrrole formation from glycine and succinyl-CoA, negative regulation of tetrapyrrole synthesis from glycine and succinyl-CoA, inhibition of tetrapyrrole biosynthetic process from glycine and succinyl-CoA Relationships: is a type of negative regulation of amide metabolic process [GO:0034249]; is a type of GO:0045763; is a type of negative regulation of nucleobase-containing compound metabolic process [GO:0045934]; is a type of GO:0045936; is a type of negative regulation of small molecule metabolic process [GO:0062014]; is a type of regulation of tetrapyrrole biosynthetic process from glycine and succinyl-CoA [GO:1901413]; is a type of negative regulation of tetrapyrrole biosynthetic process [GO:1901464]; negatively regulates tetrapyrrole biosynthetic process from glycine and succinyl-CoA [GO:0033527] Definition: Any process that stops, prevents or reduces the frequency, rate or extent of tetrapyrrole biosynthetic process from glycine and succinyl-CoA.